{
  "gene_symbol": "CEP295",
  "term_label": "cytosol",
  "gene": "UniProtKB:Q9C0D2",
  "term_id": "GO:0005829",
  "gene_name": "Centrosomal protein of 295 kDa"
}